conidium germination [GO:0120164] (biological process) Definition: The physiological and developmental changes that occur in a conidium or asexual spore following release from dormancy up to the earliest signs of development such as swelling of conidia, adhesion and nuclear decondensation followed by hyphal growth several hours later. In many genera of plant pathogenic fungi (e.g. Magnaporthe, Colletotrichum, Ustilago), swelling of the hyphal tips to form appressorium, metabolic activities including respiration, RNA and protein synthesis and trehalose breakdown and changes in cell wall composition can be detected in conidium germination. References: PMID:10835388, PMID:11377860, PMID:17950638, PMID:18944978, PMID:25063657, PMID:27355215, PMID:9529886 Sources: DOI:10.1128/9781555815523.ch10 Relationships: is a type of GO:0009847